{
  "gene": "UniProtKB:Q15459",
  "gene_symbol": "SF3A1",
  "term_id": "GO:0003723",
  "gene_name": "Splicing factor 3A subunit 1",
  "term_label": "RNA binding"
}